low-density lipoprotein particle clearance [GO:0034383] (biological process) Regulation: regulated by regulation of low-density lipoprotein particle clearance [GO:0010988]; negatively regulated by negative regulation of low-density lipoprotein particle clearance [GO:0010989]; positively regulated by positive regulation of low-density lipoprotein particle clearance [GO:1905581] Relationships: is a type of plasma lipoprotein particle clearance [GO:0034381]; has part low-density lipoprotein particle disassembly [GO:0090495] Definition: The process in which a low-density lipoprotein particle is removed from the blood via receptor-mediated endocytosis and its constituent parts degraded. Sources: GOC:BHF, GOC:mah Also known as: LDL clearance